regulation of sebum secreting cell proliferation [GO:1904002] (biological process) Also known as: regulation of sebocyte proliferation References: PMID:16901790 Sources: GOC:TermGenie, GOC:hjd, GO_REF:0000058 Relationships: is a type of regulation of epithelial cell proliferation [GO:0050678]; regulates sebum secreting cell proliferation [GO:1990654] Definition: Any process that modulates the frequency, rate or extent of sebum secreting cell proliferation. Subtypes: GO:1904003, positive regulation of sebum secreting cell proliferation [GO:1904004]